cell wall macromolecule catabolic process involved in cell wall disassembly [GO:0070910] (biological process) Sources: GOC:mah Subtypes: GO:0071854 Definition: The chemical reactions and pathways that result in the breakdown of macromolecules that form part of a cell wall, and contributes to the breakdown of the cell wall. Relationships: is a type of cell wall macromolecule catabolic process [GO:0016998]; is part of cell wall disassembly [GO:0044277]